negative regulation of adipose tissue development [GO:1904178] (BP) Definition: Any process that stops, prevents or reduces the frequency, rate or extent of adipose tissue development. Relationships: is a type of negative regulation of developmental process [GO:0051093]; is a type of negative regulation of multicellular organismal process [GO:0051241]; is a type of regulation of adipose tissue development [GO:1904177]; negatively regulates adipose tissue development [GO:0060612] References: PMID:23081848 Sources: GOC:TermGenie, GO_REF:0000058 Also known as: down regulation of adipose tissue development, down-regulation of adipose tissue development, downregulation of adipose tissue development, inhibition of adipose tissue development, down regulation of adipogenesis, down-regulation of adipogenesis, downregulation of adipogenesis, inhibition of adipogenesis, negative regulation of adipogenesis